death receptor binding [GO:0005123] (molecular function) References: PMID:15654015 Sources: GOC:ceb, GOC:rl Subtypes: nerve growth factor receptor binding [GO:0005163] Also known as: APO binding, DR binding, EDAR binding, FAS binding, KILLER binding, NGFR binding, TNFR1 binding, TRAIL binding, death receptor ligand, death receptor adaptor protein activity, death receptor interacting protein activity, death receptor-associated factor activity Definition: Binding to a member of the death receptor (DR) family. The DR family falls within the tumor necrosis factor receptor superfamily and is characterized by a cytoplasmic region of ~80 residues termed the death domain (DD). Relationships: is a type of GO:0032813